{
  "gene": "UniProtKB:P32019",
  "gene_name": "Type II inositol 1,4,5-trisphosphate 5-phosphatase",
  "term_id": "GO:0052658",
  "gene_symbol": "INPP5B",
  "term_label": "inositol-1,4,5-trisphosphate 5-phosphatase activity"
}